{
  "gene_name": "Protein Wnt-7a",
  "gene_symbol": "WNT7A",
  "term_label": "canonical Wnt signaling pathway",
  "term_id": "GO:0060070",
  "gene": "UniProtKB:O00755"
}